{
  "gene_name": "Protein PML",
  "term_label": "suppression of viral release by host",
  "gene_symbol": "PML",
  "gene": "UniProtKB:P29590",
  "term_id": "GO:0044790"
}